{
  "term_id": "GO:0042127",
  "gene": "UniProtKB:Q92754",
  "term_label": "regulation of cell population proliferation",
  "gene_name": "Transcription factor AP-2 gamma",
  "gene_symbol": "TFAP2C"
}